{
  "gene_symbol": "KRTAP19-6",
  "gene_name": "Keratin-associated protein 19-6",
  "gene": "UniProtKB:Q3LI70",
  "term_id": "UNKNOWN:0003",
  "term_label": "Unknown cellular component"
}